{
  "term_id": "GO:0007399",
  "gene_symbol": "GFRA3",
  "gene_name": "GDNF family receptor alpha-3",
  "gene": "UniProtKB:O60609",
  "term_label": "nervous system development"
}